{
  "term_id": "GO:0006457",
  "term_label": "protein folding",
  "gene_name": "Peptidyl-prolyl cis-trans isomerase FKBP5",
  "gene_symbol": "FKBP5",
  "gene": "UniProtKB:Q13451"
}